{
  "gene_symbol": "LUZP6",
  "term_id": "UNKNOWN:0001",
  "gene_name": "Leucine zipper protein 6",
  "term_label": "Unknown molecular function",
  "gene": "UniProtKB:Q538Z0"
}